{
  "gene_symbol": "KLHL17",
  "gene": "UniProtKB:Q6TDP4",
  "gene_name": "Kelch-like protein 17",
  "term_id": "GO:0031463",
  "term_label": "Cul3-RING ubiquitin ligase complex"
}